negative regulation of cell proliferation involved in heart valve morphogenesis [GO:0003252] (biological process) Relationships: is a type of regulation of cell proliferation involved in heart valve morphogenesis [GO:0003250]; is a type of negative regulation of cell proliferation involved in heart morphogenesis [GO:2000137]; negatively regulates cell proliferation involved in heart valve morphogenesis [GO:0003249] Sources: GOC:mtg_heart Definition: Any process that decreases the rate, frequency or extent of cell proliferation that contributes to the shaping of a heart valve.